positive regulation of metanephros development [GO:0072216] (biological process) Subtypes: metanephric renal vesicle induction [GO:0072094], GO:0072300 Sources: GOC:mtg_kidney_jan10 Relationships: is a type of regulation of metanephros development [GO:0072215]; is a type of GO:0090184; positively regulates GO:0001656 Definition: Any process that increases the rate, frequency or extent of metanephros development. Metanephros development is the process whose specific outcome is the progression of the metanephros over time, from its formation to the mature structure. The metanephros is an organ that filters the blood and excretes the end products of body metabolism in the form of urine.